{
  "gene_name": "NADPH oxidase 3",
  "gene": "UniProtKB:Q9HBY0",
  "gene_symbol": "NOX3",
  "term_id": "GO:0005886",
  "term_label": "plasma membrane"
}